{
  "term_label": "Unknown cellular component",
  "gene": "UniProtKB:Q6RVD6",
  "gene_symbol": "SPATA8",
  "gene_name": "Spermatogenesis-associated protein 8",
  "term_id": "UNKNOWN:0003"
}